determination of left/right asymmetry in lateral mesoderm [GO:0003140] (BP) Sources: GOC:mtg_heart Relationships: is a type of determination of left/right symmetry [GO:0007368]; BFO_0000050 lateral mesoderm development [GO:0048368] Definition: The establishment of the lateral mesoderm with respect to the left and right halves.